{
  "term_label": "cytoplasm",
  "gene_name": "DDB1- and CUL4-associated factor 8-like protein 2",
  "gene": "UniProtKB:P0C7V8",
  "gene_symbol": "DCAF8L2",
  "term_id": "GO:0005737"
}